{
  "term_id": "GO:0022008",
  "gene_name": "Trafficking kinesin-binding protein 2",
  "term_label": "neurogenesis",
  "gene": "UniProtKB:O60296",
  "gene_symbol": "TRAK2"
}